leucine zipper domain binding [GO:0043522] (molecular function) Also known as: leucine zipper binding Definition: Binding to a leucine zipper domain, a protein secondary structure exhibiting a periodic repetition of leucine residues at every seventh position over a distance covering eight helical turns. Relationships: is a type of LRR domain binding [GO:0030275] Sources: GOC:jl, InterPro:IPR002158